{
  "term_id": "GO:0015485",
  "gene_name": "NPC intracellular cholesterol transporter 2",
  "gene_symbol": "NPC2",
  "gene": "UniProtKB:P61916",
  "term_label": "cholesterol binding"
}